{
  "term_label": "pattern recognition receptor activity",
  "term_id": "GO:0038187",
  "gene_symbol": "CLEC4F",
  "gene_name": "C-type lectin domain family 4 member F",
  "gene": "UniProtKB:Q8N1N0"
}